high density lipoprotein particle mediated signaling [GO:0055097] (BP) Definition: The series of molecular signals mediated by the detection of high density lipoprotein particle. Relationships: is a type of lipoprotein particle mediated signaling [GO:0055095]; is part of GO:0071403 Sources: GOC:BHF, GOC:rl Also known as: high density lipoprotein mediated signalling, high density lipoprotein particle mediated signal transduction, high density lipoprotein particle-mediated signaling